UDP-N-acetylmuramoylpentapeptide-lysine N6-alanyltransferase activity [GO:0047206] (molecular function) Definition: Catalysis of the reaction: UDP-N-acetylmuramoyl-L-alanyl-D-glutamyl-L-lysyl-D-alanyl-D-alanine + L-alanyl-tRNA(Ala) = UDP-N-acetylmuramoyl-L-alanyl-D-glutamyl-N6-(L-alanyl)-L-lysyl-D-alanyl-D-alanine + tRNA(Ala). Sources: EC:2.3.2.10 Relationships: is a type of GO:0016755 Also known as: UDP-N-acetylmuramoylpentapeptide lysine N(6)-alanyltransferase activity, UDP-N-acetylmuramoylpentapeptide lysine N6-alanyltransferase activity, alanyl-transfer ribonucleate-uridine diphosphoacetylmuramoylpentapeptide transferase activity, uridine diphosphoacetylmuramoylpentapeptide lysine N(6)-alanyltransferase activity, uridine diphosphoacetylmuramoylpentapeptide lysine N6-alanyltransferase activity